{
  "term_id": "GO:0005794",
  "gene_symbol": "GALNT8",
  "term_label": "Golgi apparatus",
  "gene_name": "Probable polypeptide N-acetylgalactosaminyltransferase 8",
  "gene": "UniProtKB:Q9NY28"
}